{
  "gene": "UniProtKB:Q8NFJ6",
  "term_label": "G protein-coupled receptor signaling pathway",
  "gene_name": "Prokineticin receptor 2",
  "term_id": "GO:0007186",
  "gene_symbol": "PROKR2"
}